{
  "gene": "UniProtKB:Q70EL2",
  "gene_symbol": "USP45",
  "term_id": "UNKNOWN:0001",
  "term_label": "Unknown molecular function",
  "gene_name": "Ubiquitin carboxyl-terminal hydrolase 45"
}